{
  "gene_name": "Undifferentiated embryonic cell transcription factor 1",
  "gene": "UniProtKB:Q5T230",
  "term_id": "GO:0005634",
  "gene_symbol": "UTF1",
  "term_label": "nucleus"
}